{
  "gene_name": "Aquaporin-11",
  "term_id": "GO:0015267",
  "term_label": "channel activity",
  "gene": "UniProtKB:Q8NBQ7",
  "gene_symbol": "AQP11"
}